{
  "gene": "UniProtKB:Q6PIF2",
  "term_label": "Unknown molecular function",
  "term_id": "UNKNOWN:0001",
  "gene_name": "Synaptonemal complex central element protein 2",
  "gene_symbol": "SYCE2"
}